6-methylsalicylate decarboxylase activity [GO:0047596] (molecular function) Relationships: is a type of GO:0016831 Also known as: 6-MSA decarboxylase activity, 6-methylsalicylate carboxy-lyase (3-cresol-forming), 6-methylsalicylate carboxy-lyase activity, 6-methylsalicylic acid (2,6-cresotic acid) decarboxylase activity Sources: EC:4.1.1.52, RHEA:23112 Definition: Catalysis of the reaction: 6-methylsalicylate + H+ = 3-cresol + CO2.